{
  "term_id": "GO:0004674",
  "gene_name": "Mitogen-activated protein kinase 4",
  "term_label": "protein serine/threonine kinase activity",
  "gene_symbol": "MAPK4",
  "gene": "UniProtKB:P31152"
}